{
  "gene_name": "MAP kinase-activated protein kinase 3",
  "gene": "UniProtKB:Q16644",
  "term_id": "GO:0005737",
  "gene_symbol": "MAPKAPK3",
  "term_label": "cytoplasm"
}